{
  "gene_name": "Zinc finger protein with KRAB and SCAN domains 8",
  "gene": "UniProtKB:Q15776",
  "gene_symbol": "ZKSCAN8",
  "term_label": "DNA-binding transcription factor activity, RNA polymerase II-specific",
  "term_id": "GO:0000981"
}